o-orsellinic acid catabolic process [GO:1900583] (biological process) Also known as: o-orsellinic acid breakdown, o-orsellinic acid catabolism, o-orsellinic acid degradation Definition: The chemical reactions and pathways resulting in the breakdown of o-orsellinic acid. Sources: GOC:TermGenie, GOC:di Relationships: is a type of phenol-containing compound catabolic process [GO:0019336]; is a type of GO:0042537; is a type of GO:0072329; is a type of secondary metabolite catabolic process [GO:0090487]